ethanolamine-phosphate cytidylyltransferase activity [GO:0004306] (molecular function) Sources: EC:2.7.7.14 Also known as: phosphorylethanolamine transferase activity, CTP:ethanolamine-phosphate cytidylyltransferase activity, phosphoethanolamine cytidylyltransferase activity, CTP-phosphoethanolamine cytidylyltransferase activity, CTP:phosphoethanolamine cytidylyltransferase activity, ET, ethanolamine phosphate cytidylyltransferase activity Relationships: is a type of cytidylyltransferase activity [GO:0070567] Definition: Catalysis of the reaction: CTP + ethanolamine phosphate = diphosphate + CDP-ethanolamine.